{
  "term_label": "acetylcholine-gated monoatomic cation-selective channel activity",
  "term_id": "GO:0022848",
  "gene": "UniProtKB:Q494W8",
  "gene_symbol": "CHRFAM7A",
  "gene_name": "CHRNA7-FAM7A fusion protein"
}